symbiont-mediated suppression of host autophagy [GO:0140321] (biological process) Definition: A process in which a symbiont inhibits or disrupts the normal execution of autophagy in the host cell. The host is defined as the larger of the organisms involved in a symbiotic interaction. Sources: GOC:pg Also known as: negative regulation by symbiont of host autophagy, suppression of host autophagy Relationships: is a type of symbiont-mediated perturbation of host autophagy [GO:0075071]